nicotinamide N-methyltransferase activity [GO:0008112] (molecular function) Also known as: S-adenosyl-L-methionine:nicotinamide N-methyltransferase activity, nicotinamide methyltransferase activity Sources: EC:2.1.1.1, RHEA:23884 Relationships: is a type of N-methyltransferase activity [GO:0008170]; is a type of S-adenosylmethionine-dependent methyltransferase activity [GO:0008757] Definition: Catalysis of the reaction: S-adenosyl-L-methionine(1+) + nicotinamide = 1-methylnicotinamide + S-adenosyl-L-homocysteine.